synaptic vesicle endocytosis [GO:0048488] (biological process) Definition: A vesicle-mediated transport process, in which the synaptic vesicle membrane constituents are retrieved from the presynaptic membrane on the axon terminal after neurotransmitter secretion by exocytosis. Synaptic vesicle endocytosis can occur via clathrin-dependent and clathrin-independent mechanisms. Relationships: is a type of presynaptic endocytosis [GO:0140238]; is part of synaptic vesicle recycling [GO:0036465] Subtypes: clathrin-dependent synaptic vesicle endocytosis [GO:0150007], GO:0150008 References: PMID:20448150, PMID:26430111 Sources: GOC:aruk, GOC:bc, GOC:jid, GOC:lmg, GOC:mah Also known as: synaptic vesicle retrieval Regulation: regulated by regulation of synaptic vesicle endocytosis [GO:1900242]; negatively regulated by negative regulation of synaptic vesicle endocytosis [GO:1900243]; positively regulated by GO:1900244